{
  "term_id": "GO:0006511",
  "gene": "UniProtKB:Q6ZMZ0",
  "gene_name": "E3 ubiquitin-protein ligase RNF19B",
  "gene_symbol": "RNF19B",
  "term_label": "ubiquitin-dependent protein catabolic process"
}